{
  "gene_symbol": "ARMCX6",
  "term_id": "GO:0019896",
  "gene": "UniProtKB:Q7L4S7",
  "gene_name": "Protein ARMCX6",
  "term_label": "axonal transport of mitochondrion"
}